AMP nucleosidase activity [GO:0008714] (molecular function) Definition: Catalysis of the reaction: AMP + H2O = D-ribose 5-phosphate + adenine. Sources: EC:3.2.2.4, RHEA:20129 Also known as: AMP phosphoribohydrolase activity, adenosine monophosphate nucleosidase activity, adenylate nucleosidase activity Relationships: is a type of hydrolase activity, hydrolyzing N-glycosyl compounds [GO:0016799]